{
  "gene": "UniProtKB:Q6ZT62",
  "term_id": "GO:0035020",
  "term_label": "regulation of Rac protein signal transduction",
  "gene_symbol": "BARGIN",
  "gene_name": "Bargin"
}